{
  "term_id": "GO:0005737",
  "gene_symbol": "CRK",
  "gene": "UniProtKB:P46108",
  "term_label": "cytoplasm",
  "gene_name": "Adapter molecule crk"
}